{
  "gene": "UniProtKB:P25490",
  "term_label": "regulation of transcription by RNA polymerase II",
  "term_id": "GO:0006357",
  "gene_symbol": "YY1",
  "gene_name": "Transcriptional repressor protein YY1"
}